{
  "term_label": "Golgi apparatus",
  "gene": "UniProtKB:Q93063",
  "gene_symbol": "EXT2",
  "gene_name": "Exostosin-2",
  "term_id": "GO:0005794"
}